{
  "term_id": "UNKNOWN:0001",
  "gene": "UniProtKB:Q3LI72",
  "gene_name": "Keratin-associated protein 19-5",
  "term_label": "Unknown molecular function",
  "gene_symbol": "KRTAP19-5"
}